{
  "term_id": "GO:0004175",
  "gene_symbol": "PSMB11",
  "gene_name": "Proteasome subunit beta type-11",
  "term_label": "endopeptidase activity",
  "gene": "UniProtKB:A5LHX3"
}